{
  "gene": "UniProtKB:O14718",
  "term_id": "GO:0071482",
  "gene_name": "Visual pigment-like receptor peropsin",
  "gene_symbol": "RRH",
  "term_label": "cellular response to light stimulus"
}